{
  "term_label": "RNA polymerase II cis-regulatory region sequence-specific DNA binding",
  "gene": "UniProtKB:Q8N5A5",
  "gene_symbol": "ZGPAT",
  "gene_name": "Zinc finger CCCH-type with G patch domain-containing protein",
  "term_id": "GO:0000978"
}